viral inner membrane [GO:0039641] (cellular component) Also known as: virion inner membrane Definition: The lipid bilayer of a virion contained inside the protein capsid. References: PMID:15331712 Sources: GOC:bm Relationships: is a type of GO:0036338